auxin efflux carrier complex [GO:0009921] (cellular component) Definition: The protein complex associated with the plasma membrane of certain plant cells (e.g. root cortex, epidermal cells) that functions to transport auxin out of the cell. References: PMID:9843496 Relationships: is a type of plasma membrane protein complex [GO:0098797]